{
  "gene_name": "BTB_POZ domain-containing protein KCTD19",
  "gene": "UniProtKB:Q17RG1",
  "gene_symbol": "KCTD19",
  "term_label": "Unknown cellular component",
  "term_id": "UNKNOWN:0003"
}